{
  "term_label": "ubiquitin-independent protein catabolic process via the multivesicular body sorting pathway",
  "gene_name": "Vacuolar protein sorting-associated protein 4B",
  "term_id": "GO:0090611",
  "gene_symbol": "VPS4B",
  "gene": "UniProtKB:O75351"
}